{
  "term_label": "Golgi membrane",
  "term_id": "GO:0000139",
  "gene_name": "Mannosyl-oligosaccharide 1,2-alpha-mannosidase IB",
  "gene": "UniProtKB:O60476",
  "gene_symbol": "MAN1A2"
}